endocardial cushion to mesenchymal transition [GO:0090500] (BP) Subtypes: endocardial cushion to mesenchymal transition involved in heart valve formation [GO:0003199], endocardial cushion to mesenchymal transition involved in heart chamber septation [GO:0003200], GO:0003202 Definition: A transition where an endocardial cushion cell loses apical/basolateral polarity, severs intercellular adhesive junctions, degrades basement membrane components and becomes a migratory mesenchymal cell. Regulation: regulated by regulation of endocardial cushion to mesenchymal transition [GO:0140049]; negatively regulated by negative regulation of endocardial cushion to mesenchymal transition [GO:0140050]; positively regulated by positive regulation of endocardial cushion to mesenchymal transition [GO:0140051] Relationships: is a type of cardiac epithelial to mesenchymal transition [GO:0060317] Sources: GOC:dph, GOC:tb